{
  "gene": "UniProtKB:Q9Y6M5",
  "term_label": "detoxification of zinc ion",
  "gene_name": "Proton-coupled zinc antiporter SLC30A1",
  "term_id": "GO:0010312",
  "gene_symbol": "SLC30A1"
}